{
  "term_label": "Unknown biological process",
  "gene": "UniProtKB:Q9H8E8",
  "term_id": "UNKNOWN:0002",
  "gene_symbol": "KAT14",
  "gene_name": "Cysteine-rich protein 2-binding protein"
}